{
  "term_id": "GO:0003823",
  "gene_symbol": "IGHV1-45",
  "gene": "UniProtKB:A0A0A0MS14",
  "gene_name": "Immunoglobulin heavy variable 1-45",
  "term_label": "antigen binding"
}